{
  "term_label": "endocytic recycling",
  "gene_symbol": "DENND1C",
  "term_id": "GO:0032456",
  "gene_name": "DENN domain-containing protein 1C",
  "gene": "UniProtKB:Q8IV53"
}